NPHP complex [GO:1990957] (CC) Relationships: is a type of GO:0032991; is part of ciliary transition zone [GO:0035869] Also known as: NPHP module Note: Although there is some evidence, it's still unclear if the MKS and NPHP complexes are constituent parts of the ciliary Y-shaped links or are simply responsible for aligning and attaching the Y-shaped links to the cilium membrane and axoneme. Definition: A protein complex that is located at the ciliary transition zone and consists of the NPHP4 and NPHP1 proteins. It acts as an organiser of the transition zone inner structure, specifically the Y-shaped links, in conjunction with the MKS complex. It is involved in ciliary protein trafficking and is required for correct functioning of the WNT and Hippo signaling pathways. References: PMID:18337471, PMID:21422230, PMID:21498478, PMID:21555462, PMID:25150219 Sources: GOC:cilia